{
  "term_label": "Unknown biological process",
  "gene_name": "T cell receptor alpha joining 23 (Fragment)",
  "gene_symbol": "TRAJ23",
  "gene": "UniProtKB:A0A075B6U7",
  "term_id": "UNKNOWN:0002"
}